{
  "gene": "UniProtKB:Q8IZM9",
  "term_label": "L-glutamine transmembrane transporter activity",
  "gene_name": "Probable sodium-coupled neutral amino acid transporter 6",
  "gene_symbol": "SLC38A6",
  "term_id": "GO:0015186"
}